{
  "term_id": "GO:0030509",
  "term_label": "BMP signaling pathway",
  "gene_name": "Mothers against decapentaplegic homolog 6",
  "gene_symbol": "SMAD6",
  "gene": "UniProtKB:O43541"
}